{
  "term_label": "Unknown biological process",
  "gene_name": "Large ribosomal subunit protein bL34m",
  "term_id": "UNKNOWN:0002",
  "gene_symbol": "MRPL34",
  "gene": "UniProtKB:Q9BQ48"
}